{
  "term_label": "DNA-binding transcription repressor activity, RNA polymerase II-specific",
  "gene": "UniProtKB:Q8IUE0",
  "term_id": "GO:0001227",
  "gene_symbol": "TGIF2LY",
  "gene_name": "Homeobox protein TGIF2LY"
}